{
  "term_label": "Unknown molecular function",
  "gene_symbol": "LRRC46",
  "gene_name": "Leucine-rich repeat-containing protein 46",
  "gene": "UniProtKB:Q96FV0",
  "term_id": "UNKNOWN:0001"
}